regulation of mitochondrial membrane permeability involved in apoptotic process [GO:1902108] (biological process) Definition: Any regulation of mitochondrial membrane permeability that is involved in apoptotic process. References: PMID:19168129 Sources: GOC:TermGenie, GOC:mtg_apoptosis, GOC:pm Also known as: regulation of mitochondrial membrane permeability involved in apoptotic cell death, regulation of mitochondrial membrane permeability involved in apoptotic programmed cell death, regulation of mitochondrial membrane permeability involved in programmed cell death by apoptosis, regulation of transport across mitochondrial membrane involved in apoptotic cell death, regulation of transport across mitochondrial membrane involved in apoptotic process, regulation of transport across mitochondrial membrane involved in apoptotic programmed cell death, regulation of transport across mitochondrial membrane involved in programmed cell death by apoptosis, regulation of mitochondrial membrane permeability involved in apoptosis, regulation of mitochondrial membrane permeability involved in apoptotic program, regulation of mitochondrial membrane permeability involved in type I programmed cell death, regulation of transport across mitochondrial membrane involved in apoptosis, regulation of transport across mitochondrial membrane involved in apoptotic program, regulation of transport across mitochondrial membrane involved in type I programmed cell death, regulation of mitochondrial membrane permeability involved in signaling (initiator) caspase activity, regulation of transport across mitochondrial membrane involved in signaling (initiator) caspase activity Relationships: is a type of apoptotic mitochondrial changes [GO:0008637]; is a type of regulation of mitochondrial membrane permeability [GO:0046902] Subtypes: negative regulation of mitochondrial membrane permeability involved in apoptotic process [GO:1902109], positive regulation of mitochondrial membrane permeability involved in apoptotic process [GO:1902110]